{
  "gene_symbol": "ARVCF",
  "gene_name": "Splicing regulator ARVCF",
  "term_label": "cadherin binding",
  "gene": "UniProtKB:O00192",
  "term_id": "GO:0045296"
}